{
  "term_label": "translation elongation factor activity",
  "term_id": "GO:0003746",
  "gene_name": "Elongation factor Tu, mitochondrial",
  "gene": "UniProtKB:P49411",
  "gene_symbol": "TUFM"
}